{
  "term_id": "GO:0098887",
  "term_label": "neurotransmitter receptor transport, endosome to postsynaptic membrane",
  "gene_name": "Glutamate receptor-interacting protein 1",
  "gene": "UniProtKB:Q9Y3R0",
  "gene_symbol": "GRIP1"
}